{
  "term_id": "GO:0003723",
  "gene_name": "Exportin-5",
  "term_label": "RNA binding",
  "gene": "UniProtKB:Q9HAV4",
  "gene_symbol": "XPO5"
}